{
  "gene_symbol": "PSME4",
  "gene_name": "Proteasome activator complex subunit 4",
  "term_label": "spermatoproteasome complex",
  "term_id": "GO:1990111",
  "gene": "UniProtKB:Q14997"
}